{
  "term_id": "UNKNOWN:0003",
  "gene_name": "Synaptojanin-2-binding protein",
  "gene_symbol": "SYNJ2BP",
  "gene": "UniProtKB:P57105",
  "term_label": "Unknown cellular component"
}